{
  "gene_name": "Myozenin-3",
  "term_label": "FATZ binding",
  "gene_symbol": "MYOZ3",
  "gene": "UniProtKB:Q8TDC0",
  "term_id": "GO:0051373"
}